APC-IQGAP1-Rac1 complex [GO:0034745] (cellular component) Relationships: is a type of intracellular protein-containing complex [GO:0140535]; is a type of GTPase complex [GO:1905360]; is part of cell leading edge [GO:0031252] Definition: A protein complex that contains the tumor suppressor protein adenomatous polyposis coli (APC), the small GTPase Rac1, and the Rac1 and Cdc42 effector IQGAP1; may play a role in cytoskeleton organization and cell migration. References: PMID:15572129 Note: Note that the gene/protein name 'APC' should not be confused with the abbreviation for 'anaphase promoting complex'.